voltage-gated potassium channel activity involved in Purkinje myocyte action potential repolarization [GO:0086088] (molecular function) Definition: Enables the transmembrane transfer of a potassium ion by a voltage-gated channel through the plasma membrane of a Purkinje myocyte contributing to the repolarization phase of an action potential. A voltage-gated channel is a channel whose open state is dependent on the voltage across the membrane in which it is embedded. Relationships: is a type of GO:0086008; is part of GO:0086051 Sources: GOC:BHF, GOC:mtg_cardiac_conduct_nov11